{
  "term_label": "DNA helicase activity",
  "gene": "UniProtKB:Q96FC9",
  "gene_name": "ATP-dependent DNA helicase DDX11",
  "gene_symbol": "DDX11",
  "term_id": "GO:0003678"
}